ooplasm [GO:1990917] (cellular component) Relationships: is a type of GO:0005737 Definition: The cytoplasm of an ovum. References: PMID:19022436